{
  "gene": "UniProtKB:P13533",
  "gene_symbol": "MYH6",
  "term_label": "Unknown biological process",
  "term_id": "UNKNOWN:0002",
  "gene_name": "Myosin-6"
}